{
  "term_id": "GO:0004984",
  "term_label": "olfactory receptor activity",
  "gene_symbol": "OR10AD1",
  "gene": "UniProtKB:Q8NGE0",
  "gene_name": "Olfactory receptor 10AD1"
}